{
  "term_label": "potassium ion import across plasma membrane",
  "term_id": "GO:1990573",
  "gene_symbol": "ATP1A3",
  "gene_name": "Sodium_potassium-transporting ATPase subunit alpha-3",
  "gene": "UniProtKB:P13637"
}